renal protein absorption [GO:0097017] (biological process) References: PMID:18431508 Sources: GOC:yaf Definition: A renal system process in which proteins are taken up from the collecting ducts, glomerulus and proximal and distal loops of the nephron. In non-mammalian species, absorption may occur in related structures (e.g. protein absorption is observed in nephrocytes in Drosophila, see PMID:23264686). Subtypes: renal albumin absorption [GO:0097018] Relationships: is a type of GO:0070293